{
  "gene": "UniProtKB:P01133",
  "gene_symbol": "EGF",
  "term_id": "GO:0008083",
  "term_label": "growth factor activity",
  "gene_name": "Pro-epidermal growth factor"
}